creatine biosynthetic process [GO:0006601] (biological process) Sources: GOC:mah, MetaCyc:GLYCGREAT-PWY Definition: The chemical reactions and pathways resulting in the formation of creatine, N-[amino(imino)methyl]-N-methylglycine. Creatine is formed by a process beginning with amidino group transfer from L-arginine to glycine to form guanidinoacetate, followed by methyl group transfer from S-adenosyl-L-methionine to guanidinoacetate; it is then is phosphorylated to form a pool that stores high energy phosphate for the replenishment of ATP during periods of high, or fluctuating energy demand. In animals, most creatine is transported to and used in muscle. Also known as: creatine anabolism, creatine biosynthesis, creatine formation, creatine synthesis Relationships: is a type of creatine metabolic process [GO:0006600]; is a type of modified amino acid biosynthetic process [GO:0042398]; is a type of monocarboxylic acid biosynthetic process [GO:0072330]